{
  "term_label": "spindle microtubule",
  "gene_symbol": "SKA3",
  "gene": "UniProtKB:Q8IX90",
  "term_id": "GO:0005876",
  "gene_name": "Spindle and kinetochore-associated protein 3"
}